{
  "gene": "UniProtKB:Q8NFT6",
  "term_label": "protein serine/threonine kinase activator activity",
  "gene_name": "Protein DBF4 homolog B",
  "term_id": "GO:0043539",
  "gene_symbol": "DBF4B"
}